rhombomere 4 morphogenesis [GO:0021661] (biological process) Relationships: is a type of rhombomere morphogenesis [GO:0021593]; is part of rhombomere 4 development [GO:0021570] Definition: The process in which the anatomical structure of rhombomere 4 is generated and organized. Rhombomeres are transverse segments of the developing rhombencephalon. Rhombomeres are lineage restricted, express different genes from one another, and adopt different developmental fates. Rhombomeres are numbered in an anterior to posterior order. Sources: GOC:cls, GOC:curators, GOC:dgh, GOC:dph, GOC:jid